{
  "gene": "UniProtKB:Q9BT25",
  "term_id": "GO:0005813",
  "term_label": "centrosome",
  "gene_symbol": "HAUS8",
  "gene_name": "HAUS augmin-like complex subunit 8"
}